response to vasopressin [GO:1904116] (biological process) Definition: Any process that results in a change in state or activity of a cell or an organism (in terms of movement, secretion, enzyme production, gene expression, etc.) as a result of a vasopressin stimulus. Subtypes: cellular response to vasopressin [GO:1904117] Relationships: is a type of response to peptide hormone [GO:0043434] References: PMID:22811487 Sources: GOC:TermGenie, GO_REF:0000071